{
  "gene_name": "Linker for activation of T-cells family member 1",
  "term_label": "inflammatory response",
  "gene_symbol": "LAT",
  "gene": "UniProtKB:O43561",
  "term_id": "GO:0006954"
}